{
  "term_id": "GO:0004591",
  "gene_name": "2-oxoglutarate dehydrogenase-like, mitochondrial",
  "gene_symbol": "OGDHL",
  "gene": "UniProtKB:Q9ULD0",
  "term_label": "oxoglutarate dehydrogenase (succinyl-transferring) activity"
}